meiotic DNA recombinase assembly involved in reciprocal meiotic recombination [GO:0010772] (biological process) Relationships: is_a meiotic DNA recombinase assembly [GO:0000707]; is part of reciprocal meiotic recombination [GO:0007131] Definition: The aggregation, arrangement and bonding together of strand exchange proteins (recombinases) to form higher order oligomers on single-stranded DNA resulting in meiotic recombination. Meiotic recombination is the cell cycle process in which double strand breaks are formed and repaired through a double Holliday junction intermediate. Sources: GOC:dph, GOC:tb